positive regulation of follicle-stimulating hormone secretion [GO:0046881] (biological process) Sources: GOC:ai Definition: Any process that activates or increases the frequency, rate or extent of the regulated release of follicle-stimulating hormone. Also known as: positive regulation of follicle stimulating hormone secretion, up regulation of follicle-stimulating hormone secretion, up-regulation of follicle-stimulating hormone secretion, upregulation of follicle-stimulating hormone secretion, activation of follicle-stimulating hormone secretion, stimulation of follicle-stimulating hormone secretion Relationships: is a type of GO:0032278; is_a regulation of follicle-stimulating hormone secretion [GO:0046880]; positively regulates GO:0046884